leaf shaping [GO:0010358] (biological process) Also known as: leaf structural organization Definition: The developmental process that pertains to the organization of a leaf in three-dimensional space once the structure has initially formed. Relationships: is_a GO:0048532; is part of leaf morphogenesis [GO:0009965] References: PMID:16971475 Sources: GOC:tb